{
  "gene_name": "Basic salivary proline-rich protein 4",
  "gene_symbol": "PRB4",
  "gene": "UniProtKB:P10163",
  "term_label": "Unknown cellular component",
  "term_id": "UNKNOWN:0003"
}